positive regulation of mitotic actomyosin contractile ring contraction [GO:1903473] (biological process) Definition: Any process that activates or increases the frequency, rate or extent of mitotic actomyosin contractile ring contraction. References: PMID:1234 Sources: GOC:TermGenie, GOC:mtg_cell_cycle, GO_REF:0000058 Also known as: positive regulation of contractile ring contraction involved in cell cycle cytokinesis involved in mitotic cell cycle, positive regulation of cytokinesis, actomyosin ring contraction involved in mitotic cell cycle, positive regulation of mitotic actomyosin contractile ring constriction, up regulation of contractile ring contraction involved in cell cycle cytokinesis involved in mitotic cell cycle, up regulation of cytokinesis, actomyosin ring contraction involved in mitotic cell cycle, up regulation of mitotic actomyosin contractile ring contraction, up-regulation of contractile ring contraction involved in cell cycle cytokinesis involved in mitotic cell cycle, up-regulation of cytokinesis, actomyosin ring contraction involved in mitotic cell cycle, up-regulation of mitotic actomyosin contractile ring contraction, upregulation of contractile ring contraction involved in cell cycle cytokinesis involved in mitotic cell cycle, upregulation of cytokinesis, actomyosin ring contraction involved in mitotic cell cycle, upregulation of mitotic actomyosin contractile ring contraction, activation of contractile ring contraction involved in cell cycle cytokinesis involved in mitotic cell cycle, activation of cytokinesis, actomyosin ring contraction involved in mitotic cell cycle, activation of mitotic actomyosin contractile ring contraction Relationships: is a type of positive regulation of cytoskeleton organization [GO:0051495]; is a type of positive regulation of mitotic cytokinetic process [GO:1903438]; is a type of GO:1903471; positively regulates mitotic actomyosin contractile ring contraction [GO:1902404]